protein-macromolecule adaptor activity [GO:0030674] (molecular function) Also known as: protein complex scaffold activity, protein-containing complex scaffold activity, protein binding, bridging, protein-protein adaptor, protein recruiting activity Definition: An adaptor activity that brings together two or more macromolecules in contact, permitting those molecules to function in a coordinated way. The adaptor can bring together two proteins, or a protein and another macromolecule such as a lipid or a nucleic acid. Sources: GOC:bf, GOC:mah, GOC:vw Relationships: is_a molecular adaptor activity [GO:0060090]; has part protein binding [GO:0005515] Subtypes: RNA polymerase II sequence-specific DNA-binding transcription factor recruiting activity [GO:0001010], RNA polymerase II complex recruiting activity [GO:0001139], GO:0003712, guanyl-nucleotide exchange factor adaptor activity [GO:0005091], GO:0005483, SNAP receptor activity [GO:0005484], GO:0008093, signaling adaptor activity [GO:0035591], protein-membrane adaptor activity [GO:0043495], ubiquitin-like protein reader activity [GO:0140035], centriole scaffold activity [GO:0140180], cargo adaptor activity [GO:0140312], chromatin-protein adaptor activity [GO:0140463], kinetochore adaptor activity [GO:0140483], protein-RNA adaptor activity [GO:0140517], molecular condensate scaffold activity [GO:0140693], GO:0140767, receptor clustering activity [GO:0141175], ubiquitin ligase complex scaffold activity [GO:0160072], autophagy cargo adaptor activity [GO:0160247], microtubule site clamp [GO:1990644]